{
  "gene_symbol": "PRKX",
  "gene": "UniProtKB:P51817",
  "term_id": "GO:0004691",
  "gene_name": "cAMP-dependent protein kinase catalytic subunit PRKX",
  "term_label": "cAMP-dependent protein kinase activity"
}